{
  "term_id": "UNKNOWN:0002",
  "gene_symbol": "SMIM35",
  "term_label": "Unknown biological process",
  "gene_name": "Small integral membrane protein 35",
  "gene": "UniProtKB:A0A1B0GVV1"
}